attachment of GPI anchor to protein [GO:0016255] (biological process) Sources: ISBN:0879695595 Relationships: is a type of GO:0051604; is part of GPI anchored protein biosynthesis [GO:0180046] Definition: A transamidation reaction that results in the cleavage of the polypeptide chain and the concomitant transfer of the GPI anchor to the newly formed carboxy-terminal amino acid of the anchored protein. The cleaved C-terminal contains the C-terminal GPI signal sequence of the newly synthesized polypeptide chain.